phosphatidylinositol-4-phosphate binding [GO:0070273] (molecular function) Relationships: is a type of phosphatidylinositol phosphate binding [GO:1901981] Sources: GOC:bf, GOC:mah Definition: Binding to phosphatidylinositol-4-phosphate, a derivative of phosphatidylinositol in which the inositol ring is phosphorylated at the 4' position.